{
  "gene": "UniProtKB:E5RJM6",
  "gene_symbol": "ANKRD65",
  "gene_name": "Ankyrin repeat domain-containing protein 65",
  "term_id": "UNKNOWN:0001",
  "term_label": "Unknown molecular function"
}